{
  "gene_name": "Neurotrophin-3",
  "gene_symbol": "NTF3",
  "gene": "UniProtKB:P20783",
  "term_id": "GO:0008083",
  "term_label": "growth factor activity"
}